{
  "term_label": "Unknown cellular component",
  "term_id": "UNKNOWN:0003",
  "gene": "UniProtKB:Q01196",
  "gene_symbol": "RUNX1",
  "gene_name": "Runt-related transcription factor 1"
}